regulation of vasoconstriction by epinephrine [GO:0003115] (biological process) Subtypes: GO:0003119, regulation of vasoconstriction by circulating epinephrine [GO:0003120] Relationships: is a type of regulation of vasoconstriction [GO:0019229] Definition: Any process that modulates the frequency, rate or extent of reductions in the diameter of blood vessels as a result of secretion of epinephrine into the bloodstream or released by nerve endings. Sources: GOC:mtg_cardio